chitin catabolic process to fructose 6-phosphate via glucosamine [GO:0052776] (biological process) References: PMID:15136574, PMID:16232910, PMID:16736587 Sources: GOC:bf, GOC:mengo_curators, MetaCyc:PWY-6855 Relationships: is a type of GO:0006032; is a type of acetate metabolic process [GO:0006083]; is a type of phosphate-containing compound metabolic process [GO:0006796]; is a type of organophosphate metabolic process [GO:0019637]; has part N-acetylglucosamine deacetylase activity [GO:0050119]; has part exo-1,4-beta-D-glucosaminidase activity [GO:0052761]; has part diacetylchitobiose deacetylase activity [GO:0052773] Definition: The pathway resulting in the breakdown of chitin into fructose 6-phosphate, via glucosamine; acetate is also produced during the process. Also known as: diacetylchitobiose catabolic process to glucosamine and acetate